{
  "gene_symbol": "NR1I3",
  "gene_name": "Nuclear receptor subfamily 1 group I member 3",
  "term_label": "nucleus",
  "term_id": "GO:0005634",
  "gene": "UniProtKB:Q14994"
}